{
  "gene_name": "Pannexin-3",
  "term_label": "monoatomic cation transport",
  "gene_symbol": "PANX3",
  "term_id": "GO:0006812",
  "gene": "UniProtKB:Q96QZ0"
}